{
  "gene_name": "Patatin-like phospholipase domain-containing protein 2",
  "term_id": "GO:0005737",
  "term_label": "cytoplasm",
  "gene_symbol": "PNPLA2",
  "gene": "UniProtKB:Q96AD5"
}